{
  "term_label": "L-tyrosine-2-oxoglutarate transaminase activity",
  "gene": "UniProtKB:P17735",
  "gene_symbol": "TAT",
  "term_id": "GO:0004838",
  "gene_name": "Tyrosine aminotransferase"
}